{
  "term_id": "UNKNOWN:0002",
  "gene_name": "Beta-defensin 108B",
  "gene_symbol": "DEFB108B",
  "term_label": "Unknown biological process",
  "gene": "UniProtKB:Q8NET1"
}